{
  "gene_name": "Pleckstrin homology domain-containing family G member 7",
  "term_label": "Unknown cellular component",
  "gene_symbol": "PLEKHG7",
  "gene": "UniProtKB:Q6ZR37",
  "term_id": "UNKNOWN:0003"
}